{
  "gene": "UniProtKB:P55327",
  "term_id": "GO:0005737",
  "gene_name": "Tumor protein D52",
  "term_label": "cytoplasm",
  "gene_symbol": "TPD52"
}